{
  "gene_symbol": "KCNA5",
  "gene": "UniProtKB:P22460",
  "term_label": "voltage-gated potassium channel complex",
  "term_id": "GO:0008076",
  "gene_name": "Potassium voltage-gated channel subfamily A member 5"
}